{
  "gene": "UniProtKB:O75030",
  "term_label": "RNA polymerase II cis-regulatory region sequence-specific DNA binding",
  "gene_symbol": "MITF",
  "gene_name": "Microphthalmia-associated transcription factor",
  "term_id": "GO:0000978"
}